synaptic vesicle budding from presynaptic endocytic zone membrane [GO:0016185] (biological process) Definition: Evagination of the presynaptic membrane, resulting in the formation of a new synaptic vesicle. References: PMID:10099709, PMID:20448150 Sources: GOC:curators Also known as: synaptic vesicle budding from pre-synaptic membrane, synaptic vesicle budding involved in synaptic vesicle endocytosis Relationships: is a type of synaptic vesicle budding [GO:0070142]; is part of synaptic vesicle endocytosis [GO:0048488] Regulation: regulated by regulation of synaptic vesicle budding from presynaptic endocytic zone membrane [GO:0098694]